{
  "gene_symbol": "STAG3L1",
  "gene": "UniProtKB:P0CL83",
  "term_label": "Unknown biological process",
  "term_id": "UNKNOWN:0002",
  "gene_name": "Putative STAG3-like protein 1"
}